{
  "gene_symbol": "MCM7",
  "term_label": "single-stranded DNA helicase activity",
  "gene": "UniProtKB:P33993",
  "gene_name": "DNA replication licensing factor MCM7",
  "term_id": "GO:0017116"
}